{
  "gene": "UniProtKB:Q6ZWH5",
  "gene_symbol": "NEK10",
  "term_id": "GO:1902749",
  "gene_name": "Serine_threonine-protein kinase Nek10",
  "term_label": "regulation of cell cycle G2/M phase transition"
}